corticotropin-releasing hormone receptor 2 binding [GO:0051431] (molecular function) Also known as: CRHR2 binding, type 2 corticotropin releasing factor receptor binding, type 2 corticotropin-releasing factor receptor binding, type 2 corticotropin releasing factor receptor ligand References: PMID:15134857 Relationships: is a type of corticotropin-releasing hormone receptor binding [GO:0051429] Definition: Binding to a corticotropin-releasing hormone receptor type 2 (CRHR2). The CRHR2 has several splice variants that are located in sub-cortical areas of the brain and in the periphery.